icosahedral viral capsid, collar [GO:0098031] (cellular component) Relationships: is a type of GO:0044423; BFO_0000050 icosahedral viral capsid [GO:0019030] Definition: A small disk located at the base of some icosahedral virus capsids. Sources: GOC:bm